{
  "term_label": "mRNA binding",
  "term_id": "GO:0003729",
  "gene": "UniProtKB:Q9Y5A9",
  "gene_name": "YTH domain-containing family protein 2",
  "gene_symbol": "YTHDF2"
}